{
  "term_id": "UNKNOWN:0002",
  "term_label": "Unknown biological process",
  "gene_symbol": "GOLM1",
  "gene": "UniProtKB:Q8NBJ4",
  "gene_name": "Golgi membrane protein 1"
}